{
  "gene": "UniProtKB:P35228",
  "term_id": "GO:0010181",
  "gene_name": "Nitric oxide synthase, inducible",
  "term_label": "FMN binding",
  "gene_symbol": "NOS2"
}